{
  "term_label": "phosphatidylserine exposure on apoptotic cell surface",
  "gene_name": "XK-related protein 7",
  "gene_symbol": "XKR7",
  "gene": "UniProtKB:Q5GH72",
  "term_id": "GO:0070782"
}